{
  "term_id": "GO:0000977",
  "gene": "UniProtKB:Q96QS3",
  "gene_symbol": "ARX",
  "term_label": "RNA polymerase II transcription regulatory region sequence-specific DNA binding",
  "gene_name": "Homeobox protein ARX"
}